{
  "gene_name": "FMR1 neighbor protein",
  "gene_symbol": "FMR1NB",
  "gene": "UniProtKB:Q8N0W7",
  "term_label": "Unknown molecular function",
  "term_id": "UNKNOWN:0001"
}